retroviral integrase activity [GO:0044823] (molecular function) Definition: Catalysis of the covalent insertion of double-stranded retroviral DNA into host DNA. Proceeds by an endonucleolytic cleavage at each 3'-OH extremity of the viral genome, named 3'-processing, followed by a strand transfer reaction leading to the insertion of the processed viral DNA into the target DNA by a trans-esterification mechanism. Relationships: is a type of integrase activity [GO:0008907]; is part of viral genome integration into host DNA [GO:0044826] References: PMID:19091057